{
  "term_id": "GO:0046426",
  "term_label": "negative regulation of receptor signaling pathway via JAK-STAT",
  "gene": "UniProtKB:O15524",
  "gene_name": "Suppressor of cytokine signaling 1",
  "gene_symbol": "SOCS1"
}